{
  "term_id": "GO:0005737",
  "gene_name": "Muscleblind-like protein 1",
  "gene": "UniProtKB:Q9NR56",
  "gene_symbol": "MBNL1",
  "term_label": "cytoplasm"
}